{
  "term_id": "GO:0005829",
  "gene_name": "Retinol dehydrogenase 8",
  "gene": "UniProtKB:Q9NYR8",
  "gene_symbol": "RDH8",
  "term_label": "cytosol"
}